response to L-canavanine [GO:1901354] (biological process) Sources: GOC:TermGenie Subtypes: cellular response to L-canavanine [GO:0036280] Relationships: is a type of response to amino acid [GO:0043200]; is a type of response to nitrogen compound [GO:1901698]; is a type of GO:1901700 Definition: Any process that results in a change in state or activity of a cell or an organism (in terms of movement, secretion, enzyme production, gene expression, etc.) as a result of a L-canavanine stimulus.